regulation protein catabolic process at presynapse [GO:0140251] (biological process) Note: Note that this term was created for the SynGO project, and will be obsoleted when the SynGO annotations are made in Noctua. Definition: Any process that modulates the frequency, rate or extent of the chemical reactions and pathways resulting in the breakdown of a protein at the presynapse. References: PMID:27764673 Relationships: is a type of regulation protein catabolic process at synapse [GO:0140250]; occurs in presynapse [GO:0098793]